transmembrane ascorbate ferrireductase activity [GO:0140571] (molecular function) Definition: Oxidation of Fe(3+) to Fe(2+) on the outer side of a membrane coupled to the reduction of L-ascorbate to monodehydro-L-ascorbate radical on the inner side of a membrane. Electrons get transferred across the membrane during the reaction. Relationships: is a type of GO:0015453; is a type of GO:0016722 References: PMID:16911521, PMID:24449903 Sources: RHEA:30403 Also known as: L-ascorbate-cytochrome-b5 reductase activity, L-ascorbate:ferricytochrome-b5 oxidoreductase activity, ascorbate-cytochrome b5 reductase activity